{
  "term_label": "3'-5'-RNA exonuclease activity",
  "gene_symbol": "CNOT6",
  "term_id": "GO:0000175",
  "gene": "UniProtKB:Q9ULM6",
  "gene_name": "CCR4-NOT transcription complex subunit 6"
}